{
  "term_label": "positive regulation of translational initiation",
  "gene_name": "Deleted in azoospermia protein 4",
  "gene_symbol": "DAZ4",
  "gene": "UniProtKB:Q86SG3",
  "term_id": "GO:0045948"
}